{
  "gene": "UniProtKB:A0N4Z8",
  "gene_symbol": "TRAJ9",
  "gene_name": "HCG2039779 (Fragment)",
  "term_label": "Unknown molecular function",
  "term_id": "UNKNOWN:0001"
}